{
  "term_label": "transcription initiation at RNA polymerase II promoter",
  "gene_symbol": "TAF4",
  "gene_name": "Transcription initiation factor TFIID subunit 4",
  "gene": "UniProtKB:O00268",
  "term_id": "GO:0006367"
}